{
  "gene_name": "D(1B) dopamine receptor",
  "term_label": "positive regulation of MAPK cascade",
  "gene_symbol": "DRD5",
  "term_id": "GO:0043410",
  "gene": "UniProtKB:P21918"
}